{
  "gene_name": "Programmed cell death protein 4",
  "gene": "UniProtKB:Q53EL6",
  "gene_symbol": "PDCD4",
  "term_label": "nucleus",
  "term_id": "GO:0005634"
}